{
  "gene": "UniProtKB:Q6IFH4",
  "term_label": "Unknown cellular component",
  "gene_symbol": "OR6B2",
  "term_id": "UNKNOWN:0003",
  "gene_name": "Olfactory receptor 6B2"
}